D-ribose catabolic process [GO:0019303] (biological process) Also known as: D-ribose breakdown, D-ribose catabolism, D-ribose degradation Relationships: is a type of D-ribose metabolic process [GO:0006014]; is a type of pentose catabolic process [GO:0019323] Definition: The chemical reactions and pathways resulting in the breakdown of D-ribose (ribo-pentose). Sources: ISBN:0198506732